exocytic insertion of neurotransmitter receptor to postsynaptic membrane [GO:0098967] (biological process) Relationships: is a type of GO:0006887; is a type of GO:0099072; is part of neurotransmitter receptor transport to postsynaptic membrane [GO:0098969] References: PMID:19503082 Definition: The exocytic fusion of neurotransmitter receptor containing vesicles with the postsynaptic membrane resulting in the integration of NT receptors, enabling them to participate in neurotransmitter reception. This process includes tethering and docking steps that prepare vesicles for fusion. Regulation: regulated by regulation of exocytic insertion of neurotransmitter receptor to postsynaptic membrane [GO:0099145]